{
  "term_label": "cytokine-mediated signaling pathway",
  "gene_symbol": "LILRB3",
  "gene": "UniProtKB:O75022",
  "term_id": "GO:0019221",
  "gene_name": "Leukocyte immunoglobulin-like receptor subfamily B member 3"
}